1D-1-guanidino-3-amino-1,3-dideoxy-scyllo-inositol transaminase activity [GO:0047311] (molecular function) Also known as: 1D-1-guanidino-3-amino-1,3-dideoxy-scyllo-inositol aminotransferase activity, 1D-1-guanidino-3-amino-1,3-dideoxy-scyllo-inositol:pyruvate aminotransferase activity, L-alanine-N-amidino-3-(or 5-)keto-scyllo-inosamine transaminase activity, guanidinoaminodideoxy-scyllo-inositol-pyruvate aminotransferase activity Definition: Catalysis of the reaction: 1D-1-guanidino-3-amino-1,3-dideoxy-scyllo-inositol + pyruvate = 1D-1-guanidino-1-deoxy-3-dehydro-scyllo-inositol + L-alanine. Relationships: is a type of transaminase activity [GO:0008483] Sources: EC:2.6.1.56, RHEA:15497